{
  "gene": "UniProtKB:Q8IWN7",
  "term_id": "GO:0060041",
  "gene_name": "Retinitis pigmentosa 1-like 1 protein",
  "gene_symbol": "RP1L1",
  "term_label": "retina development in camera-type eye"
}